{
  "term_id": "UNKNOWN:0001",
  "term_label": "Unknown molecular function",
  "gene": "UniProtKB:Q9NWH9",
  "gene_name": "SAFB-like transcription modulator",
  "gene_symbol": "SLTM"
}